{
  "term_id": "GO:0005634",
  "gene_name": "Zinc finger protein 852",
  "gene": "UniProtKB:Q6ZMS4",
  "gene_symbol": "ZNF852",
  "term_label": "nucleus"
}